{
  "gene_symbol": "HTT",
  "gene": "UniProtKB:P42858",
  "gene_name": "Huntingtin",
  "term_id": "GO:0048489",
  "term_label": "synaptic vesicle transport"
}